{
  "gene": "UniProtKB:P42338",
  "gene_symbol": "PIK3CB",
  "term_id": "GO:0016303",
  "gene_name": "Phosphatidylinositol 4,5-bisphosphate 3-kinase catalytic subunit beta isoform",
  "term_label": "1-phosphatidylinositol-3-kinase activity"
}